{
  "term_label": "Unknown molecular function",
  "gene_name": "Biorientation of chromosomes in cell division protein 1-like 1",
  "term_id": "UNKNOWN:0001",
  "gene_symbol": "BOD1L1",
  "gene": "UniProtKB:Q8NFC6"
}